{
  "gene_symbol": "JADE3",
  "term_label": "regulation of transcription by RNA polymerase II",
  "term_id": "GO:0006357",
  "gene_name": "Protein Jade-3",
  "gene": "UniProtKB:Q92613"
}